{
  "gene_name": "Myozenin-1",
  "gene": "UniProtKB:Q9NP98",
  "term_label": "FATZ binding",
  "gene_symbol": "MYOZ1",
  "term_id": "GO:0051373"
}